{
  "gene_name": "Selenide, water dikinase 1",
  "term_id": "GO:0005737",
  "gene_symbol": "SEPHS1",
  "gene": "UniProtKB:P49903",
  "term_label": "cytoplasm"
}